{
  "term_id": "GO:0035329",
  "gene_symbol": "AMOT",
  "term_label": "hippo signaling",
  "gene": "UniProtKB:Q4VCS5",
  "gene_name": "Angiomotin"
}